{
  "gene": "UniProtKB:Q9Y547",
  "term_label": "centrosome",
  "term_id": "GO:0005813",
  "gene_symbol": "IFT25",
  "gene_name": "Intraflagellar transport protein 25 homolog"
}